{
  "term_label": "presynaptic membrane",
  "gene": "UniProtKB:P14416",
  "term_id": "GO:0042734",
  "gene_name": "D(2) dopamine receptor",
  "gene_symbol": "DRD2"
}